{
  "term_label": "extracellular space",
  "gene_name": "Granzyme A",
  "term_id": "GO:0005615",
  "gene": "UniProtKB:P12544",
  "gene_symbol": "GZMA"
}